{
  "gene_symbol": "KIF13B",
  "gene_name": "Kinesin-like protein KIF13B",
  "term_id": "GO:0016887",
  "gene": "UniProtKB:Q9NQT8",
  "term_label": "ATP hydrolysis activity"
}